{
  "term_id": "UNKNOWN:0002",
  "gene": "UniProtKB:P61513",
  "gene_name": "Large ribosomal subunit protein eL43",
  "gene_symbol": "RPL37A",
  "term_label": "Unknown biological process"
}